{
  "term_label": "anterograde synaptic vesicle transport",
  "gene_name": "Tripartite motif-containing protein 46",
  "gene_symbol": "TRIM46",
  "gene": "UniProtKB:Q7Z4K8",
  "term_id": "GO:0048490"
}